{
  "term_label": "nucleoplasm",
  "gene_name": "Protein lin-9 homolog",
  "gene": "UniProtKB:Q5TKA1",
  "gene_symbol": "LIN9",
  "term_id": "GO:0005654"
}